{
  "term_label": "serine-type endopeptidase activity",
  "gene": "UniProtKB:P07477",
  "gene_symbol": "PRSS1",
  "gene_name": "Serine protease 1",
  "term_id": "GO:0004252"
}